{
  "gene_name": "Myosin light chain 1_3, skeletal muscle isoform",
  "term_id": "GO:0043292",
  "gene": "UniProtKB:P05976",
  "term_label": "contractile muscle fiber",
  "gene_symbol": "MYL1"
}